CD4-positive, CD25-positive, alpha-beta regulatory T cell differentiation involved in immune response [GO:0002298] (biological process) Also known as: CD4-positive, CD25-positive, alpha-beta T cell development involved in immune response, CD4-positive, CD25-positive, alpha-beta regulatory T cell differentiation during immune response, CD4-positive, CD25-positive, alpha-beta regulatory T lymphocyte differentiation during immune response, CD4-positive, CD25-positive, alpha-beta regulatory T-cell differentiation during immune response, CD4-positive, CD25-positive, alpha-beta regulatory T-lymphocyte differentiation during immune response Note: Note that immunologists typically use the word 'development' to refer to cells of B or T cell lineages undergoing the process that GO describes as 'cell differentiation'. Definition: The process in which an antigenically naive CD4-positive, alpha-beta T cell acquires the specialized features of a CD4-positive, CD25-positive, alpha-beta regulatory T cell as part of an immune response. References: PMID:12093005 Sources: GOC:add Regulation: regulated by regulation of CD4-positive, CD25-positive, alpha-beta regulatory T cell differentiation involved in immune response [GO:0032832]; negatively regulated by negative regulation of CD4-positive, CD25-positive, alpha-beta regulatory T cell differentiation involved in immune response [GO:0032833]; positively regulated by positive regulation of CD4-positive, CD25-positive, alpha-beta regulatory T cell differentiation involved in immune response [GO:0032834] Relationships: is a type of CD4-positive, alpha-beta T cell differentiation involved in immune response [GO:0002294]; is a type of CD4-positive, CD25-positive, alpha-beta regulatory T cell differentiation [GO:0002361]